{
  "term_id": "GO:0031410",
  "gene_symbol": "RUSC1",
  "gene_name": "AP-4 complex accessory subunit RUSC1",
  "gene": "UniProtKB:Q9BVN2",
  "term_label": "cytoplasmic vesicle"
}